{
  "term_label": "Unknown biological process",
  "term_id": "UNKNOWN:0002",
  "gene_symbol": "Q6ZUG5",
  "gene": "UniProtKB:Q6ZUG5",
  "gene_name": "Uncharacterized protein FLJ43738"
}